scutellarein 7-O-glucuronosyltransferase activity [GO:0102467] (molecular function) Definition: Catalysis of the reaction: scutellarein + UDP-alpha-D-glucuronate = scutellarin + UDP. Sources: RHEA:28318 Relationships: is a type of hexosyltransferase activity [GO:0016758]